ESCRT complex [GO:0036452] (cellular component) References: PMID:16689637 Sources: VZ:1536 Definition: An endosomal sorting complex involved in membrane fission processes related to sorting of multivesicular bodies (MVB) in the endocytic pathway, cytokinesis and viral budding among other processes. Also known as: endosomal sorting complex required for transport Subtypes: GO:0000813, GO:0000814, ESCRT III complex [GO:0000815], ESCRT-0 complex [GO:0033565], ESCRT IV complex [GO:1990621] Relationships: is a type of GO:0032991; BFO_0000050 endosome [GO:0005768]